1,4-alpha-oligoglucan phosphorylase activity [GO:0004645] (molecular function) Sources: RHEA:41732 Definition: Catalysis of the reaction: 1,4-alpha-D-glucosyl(n) + phosphate = 1,4-alpha-D-glucosyl(n-1) + alpha-D-glucose 1-phosphate. Relationships: is a type of hexosyltransferase activity [GO:0016758] Subtypes: glycogen phosphorylase activity [GO:0008184], GO:0009018, maltodextrin phosphorylase activity [GO:0031220], alpha,alpha-trehalose phosphorylase activity [GO:0047656], cellobiose phosphorylase activity [GO:0047738], maltose phosphorylase activity [GO:0050082], trehalose 6-phosphate phosphorylase activity [GO:0050503], glucosylglycerate phosphorylase activity [GO:0110068] Also known as: alpha-glucan phosphorylase, amylopectin phosphorylase, amylophosphorylase activity, glucan phosphorylase, glucosan phosphorylase, granulose phosphorylase, muscle phosphorylase, muscle phosphorylase a and b activity, myophosphorylase, potato phosphorylase, starch phosphorylase, 1,4-alpha-D-glucan:phosphate alpha-D-glucosyltransferase activity, 1,4-alpha-glucan phosphorylase activity, polyphosphorylase activity